{
  "gene_name": "Class A basic helix-loop-helix protein 15",
  "term_id": "GO:0070888",
  "gene_symbol": "BHLHA15",
  "gene": "UniProtKB:Q7RTS1",
  "term_label": "E-box binding"
}